DNA polymerase binding [GO:0070182] (molecular function) Relationships: is a type of enzyme binding [GO:0019899] Definition: Binding to a DNA polymerase. Sources: GOC:BHF, GOC:mah